ATP-dependent protein binding [GO:0043008] (molecular function) Sources: GOC:jl Relationships: is a type of GO:0005515 Definition: Binding to a protein or protein complex using energy from ATP hydrolysis.